keratinocyte proliferation [GO:0043616] (biological process) Definition: The multiplication or reproduction of keratinocytes, resulting in the expansion of a cell population. Keratinocytes are epidermal cells which synthesize keratin and undergo a characteristic change as they move upward from the basal layers of the epidermis to the cornified (horny) layer of the skin. Sources: CL:0000311 Regulation: regulated by GO:0010837; positively regulated by positive regulation of keratinocyte proliferation [GO:0010838]; negatively regulated by negative regulation of keratinocyte proliferation [GO:0010839] Relationships: is a type of epithelial cell proliferation [GO:0050673]